{
  "gene_symbol": "OR1J1",
  "gene": "UniProtKB:Q8NGS3",
  "gene_name": "Olfactory receptor 1J1",
  "term_id": "GO:0007165",
  "term_label": "signal transduction"
}